{
  "gene": "UniProtKB:Q9BXB1",
  "gene_symbol": "LGR4",
  "term_id": "GO:0090263",
  "gene_name": "Leucine-rich repeat-containing G-protein coupled receptor 4",
  "term_label": "positive regulation of canonical Wnt signaling pathway"
}